{
  "term_id": "GO:0050778",
  "term_label": "positive regulation of immune response",
  "gene_symbol": "HLA-DQB2",
  "gene": "UniProtKB:P05538",
  "gene_name": "HLA class II histocompatibility antigen, DQ beta 2 chain"
}